{
  "term_label": "nervous system development",
  "term_id": "GO:0007399",
  "gene_name": "Laminin subunit alpha-2",
  "gene_symbol": "LAMA2",
  "gene": "UniProtKB:P24043"
}